fin regeneration [GO:0031101] (BP) Sources: GOC:dgh Definition: The regrowth of fin tissue following its loss or destruction. Relationships: is a type of GO:0042246